{
  "term_label": "Unknown biological process",
  "gene_name": "Late cornified envelope protein 3A",
  "term_id": "UNKNOWN:0002",
  "gene": "UniProtKB:Q5TA76",
  "gene_symbol": "LCE3A"
}